CRD-mediated mRNA stability complex [GO:0070937] (cellular component) Note: See also the molecular function term 'alkyl hydroperoxide reductase activity ; GO:0008785'. References: PMID:19029303 Sources: GOC:mah Also known as: coding-region determinant of instability-mediated mRNA stability complex, coding-region instability determinant -mediated mRNA stability complex Definition: A protein complex that binds to, and promotes stabilization of, mRNA molecules containing the coding region instability determinant (CRD). In human, it may consist of IGF2BP1, HNRNPU, SYNCRIP/HNRNPQ, YBX1, and DHX9. Relationships: is a type of intracellular protein-containing complex [GO:0140535]